{
  "gene": "UniProtKB:Q9P0J1",
  "term_label": "mitochondrion",
  "gene_name": "[Pyruvate dehydrogenase [acetyl-transferring]]-phosphatase 1, mitochondrial",
  "term_id": "GO:0005739",
  "gene_symbol": "PDP1"
}